{
  "gene": "UniProtKB:Q9NSC2",
  "term_label": "DNA-binding transcription factor activity, RNA polymerase II-specific",
  "term_id": "GO:0000981",
  "gene_name": "Sal-like protein 1",
  "gene_symbol": "SALL1"
}